{
  "gene": "UniProtKB:Q9H3U1",
  "term_label": "protein folding",
  "gene_symbol": "UNC45A",
  "term_id": "GO:0006457",
  "gene_name": "Protein unc-45 homolog A"
}